{
  "term_id": "GO:0006338",
  "gene_symbol": "HMGB1P1",
  "gene_name": "Putative high mobility group protein B1-like 1",
  "gene": "UniProtKB:B2RPK0",
  "term_label": "chromatin remodeling"
}